axon guidance [GO:0007411] (biological process) Relationships: is a type of GO:0097485; is part of GO:0007409 Subtypes: motor neuron axon guidance [GO:0008045], corticospinal neuron axon guidance [GO:0021966], GO:0021967, corticospinal neuron axon guidance through the internal capsule [GO:0021968], corticospinal neuron axon guidance through the cerebral peduncle [GO:0021969], corticospinal neuron axon guidance through the basilar pons [GO:0021970], corticospinal neuron axon guidance through the medullary pyramid [GO:0021971], corticospinal neuron axon guidance through spinal cord [GO:0021972], retinal ganglion cell axon guidance [GO:0031290], dorsal/ventral axon guidance [GO:0033563], anterior/posterior axon guidance [GO:0033564], dopaminergic neuron axon guidance [GO:0036514], GO:0036515, olfactory bulb axon guidance [GO:0071678], commissural neuron axon guidance [GO:0071679], photoreceptor cell axon guidance [GO:0072499], sensory neuron axon guidance [GO:0097374], interneuron axon guidance [GO:0097376], sympathetic neuron axon guidance [GO:0097492] Regulation: regulated by GO:1902667; RO_0002212 by negative regulation of axon guidance [GO:1902668]; positively regulated by positive regulation of axon guidance [GO:1902669] Definition: The chemotaxis process that directs the migration of an axon growth cone to a specific target site in response to a combination of attractive and repulsive cues. Also known as: axon pathfinding, axon growth cone guidance, axon chemotaxis Sources: ISBN:0878932437